inductive mesenchymal to epithelial cell signaling [GO:0060522] (biological process) Relationships: is a type of inductive cell-cell signaling [GO:0031129] Also known as: inductive mesenchymal to epithelial cell signalling Definition: Signaling at short range from mesenchymal cells to cells of an epithelium that results in a developmental change in the epithelial cells. Subtypes: GO:0060521 Sources: GOC:dph